{
  "gene": "UniProtKB:P0DMW5",
  "gene_name": "Small integral membrane protein 10-like protein 2B",
  "term_label": "Unknown cellular component",
  "term_id": "UNKNOWN:0003",
  "gene_symbol": "SMIM10L2B"
}